{
  "term_label": "G protein-coupled receptor signaling pathway",
  "gene": "UniProtKB:P50150",
  "gene_name": "Guanine nucleotide-binding protein G(I)_G(S)_G(O) subunit gamma-4",
  "term_id": "GO:0007186",
  "gene_symbol": "GNG4"
}